{
  "term_label": "PRC1 complex",
  "gene_symbol": "PCGF6",
  "gene_name": "Polycomb group RING finger protein 6",
  "gene": "UniProtKB:Q9BYE7",
  "term_id": "GO:0035102"
}